{
  "term_id": "UNKNOWN:0002",
  "gene_name": "Aspartate-rich protein 1",
  "gene_symbol": "DRICH1",
  "term_label": "Unknown biological process",
  "gene": "UniProtKB:Q6PGQ1"
}